{
  "term_id": "GO:0005739",
  "gene": "UniProtKB:O75521",
  "gene_name": "Enoyl-CoA delta isomerase 2",
  "gene_symbol": "ECI2",
  "term_label": "mitochondrion"
}